{
  "term_id": "GO:0005770",
  "gene_name": "Vacuolar protein sorting-associated protein 35",
  "gene_symbol": "VPS35",
  "term_label": "late endosome",
  "gene": "UniProtKB:Q96QK1"
}